{
  "term_id": "GO:0003743",
  "gene_name": "Eukaryotic translation initiation factor 5",
  "gene": "UniProtKB:P55010",
  "gene_symbol": "EIF5",
  "term_label": "translation initiation factor activity"
}